{
  "gene": "UniProtKB:Q9NP79",
  "term_label": "late endosome to vacuole transport via multivesicular body sorting pathway",
  "term_id": "GO:0032511",
  "gene_name": "Vacuolar protein sorting-associated protein VTA1 homolog",
  "gene_symbol": "VTA1"
}